{
  "term_label": "mRNA splicing, via spliceosome",
  "term_id": "GO:0000398",
  "gene": "UniProtKB:Q12874",
  "gene_name": "Splicing factor 3A subunit 3",
  "gene_symbol": "SF3A3"
}